{
  "gene_symbol": "ATP11C",
  "term_id": "GO:0005783",
  "gene": "UniProtKB:Q8NB49",
  "gene_name": "Phospholipid-transporting ATPase IG",
  "term_label": "endoplasmic reticulum"
}